cerebellum morphogenesis [GO:0021587] (biological process) Definition: The process in which the anatomical structure of the cerebellum is generated and organized. The cerebellum is the portion of the brain in the back of the head between the cerebrum and the pons. The cerebellum controls balance for walking and standing, modulates the force and range of movement and is involved in the learning of motor skills. Relationships: is_a anatomical structure morphogenesis [GO:0009653]; is part of cerebellum development [GO:0021549]; is part of hindbrain morphogenesis [GO:0021575] Sources: GOC:cls, GOC:dgh, GOC:dph, GOC:jid, GO_REF:0000021